{
  "term_id": "UNKNOWN:0002",
  "gene_symbol": "FAM124B",
  "gene": "UniProtKB:Q9H5Z6",
  "gene_name": "Protein FAM124B",
  "term_label": "Unknown biological process"
}